regulation of Toll signaling pathway [GO:0008592] (biological process) Definition: Any process that modulates the frequency, rate or extent of the Tl signaling pathway. Relationships: is a type of regulation of signal transduction [GO:0009966]; regulates Toll signaling pathway [GO:0008063] Subtypes: negative regulation of Toll signaling pathway [GO:0045751], GO:0045752 Also known as: regulation of Tl signaling pathway, regulation of Tl signalling pathway, regulation of Toll signalling pathway Sources: GOC:go_curators